{
  "term_label": "cyclin-dependent protein kinase holoenzyme complex",
  "gene_name": "Cyclin-dependent kinase 14",
  "gene_symbol": "CDK14",
  "gene": "UniProtKB:O94921",
  "term_id": "GO:0000307"
}